{
  "term_id": "GO:0005634",
  "gene_name": "Ubiquitin-conjugating enzyme E2 E2",
  "term_label": "nucleus",
  "gene_symbol": "UBE2E2",
  "gene": "UniProtKB:Q96LR5"
}